nitroglycerin metabolic process [GO:0018937] (biological process) Also known as: NG metabolic process, NG metabolism, nitroglycerin metabolism Definition: The chemical reactions and pathways involving nitroglycerin, a well-known nitrate ester and an important component of dynamite and other propellants. Toxic to algae, invertebrate, and vertebrates. Sources: UM-BBD_pathwayID:ng Relationships: is a type of xenobiotic metabolic process [GO:0006805]